{
  "gene": "UniProtKB:Q14563",
  "gene_name": "Semaphorin-3A",
  "gene_symbol": "SEMA3A",
  "term_label": "positive regulation of cell migration",
  "term_id": "GO:0030335"
}